organosilicon catabolic process [GO:0046455] (biological process) Subtypes: GO:0046517 Sources: GOC:ai Relationships: is a type of xenobiotic catabolic process [GO:0042178] Also known as: organosilicon breakdown, organosilicon catabolism, organosilicon degradation, organosilicone catabolic process, organosilicone catabolism Definition: The chemical reactions and pathways resulting in the breakdown of organosilicons, any organic compound that contains silicon.